{
  "gene": "UniProtKB:P33527",
  "term_label": "basolateral plasma membrane",
  "gene_name": "Multidrug resistance-associated protein 1",
  "gene_symbol": "ABCC1",
  "term_id": "GO:0016323"
}